{
  "term_label": "negative regulation of cAMP/PKA signal transduction",
  "gene_symbol": "PDE4D",
  "term_id": "GO:0141162",
  "gene": "UniProtKB:Q08499",
  "gene_name": "cAMP-specific 3',5'-cyclic phosphodiesterase 4D"
}